{
  "gene_name": "Formin-2",
  "gene_symbol": "FMN2",
  "term_id": "GO:0070649",
  "gene": "UniProtKB:Q9NZ56",
  "term_label": "formin-nucleated actin cable assembly"
}